{
  "gene_symbol": "SPATA31C1",
  "gene": "UniProtKB:P0DKV0",
  "term_label": "Unknown biological process",
  "term_id": "UNKNOWN:0002",
  "gene_name": "Putative spermatogenesis-associated protein 31C1"
}